{
  "term_id": "UNKNOWN:0003",
  "term_label": "Unknown cellular component",
  "gene_symbol": "PATE3",
  "gene_name": "Prostate and testis expressed protein 3",
  "gene": "UniProtKB:B3GLJ2"
}